{
  "term_id": "GO:0035556",
  "gene_name": "PH domain leucine-rich repeat-containing protein phosphatase 1",
  "gene_symbol": "PHLPP1",
  "gene": "UniProtKB:O60346",
  "term_label": "intracellular signal transduction"
}